{
  "term_label": "Unknown molecular function",
  "gene": "UniProtKB:Q08830",
  "term_id": "UNKNOWN:0001",
  "gene_name": "Fibrinogen-like protein 1",
  "gene_symbol": "FGL1"
}